{
  "gene_symbol": "CAD",
  "term_id": "GO:0004151",
  "gene_name": "CAD protein",
  "term_label": "dihydroorotase activity",
  "gene": "UniProtKB:P27708"
}